{
  "term_id": "UNKNOWN:0001",
  "gene": "UniProtKB:Q96J88",
  "gene_name": "Epithelial-stromal interaction protein 1",
  "term_label": "Unknown molecular function",
  "gene_symbol": "EPSTI1"
}